crinophagy [GO:0160155] (biological process) References: PMID:29066608, PMID:35452619 Relationships: is a type of GO:0006914 Definition: The autophagic process which involves the direct fusion of abnormal, excess or obsolete secretory granules with lysosomes. This pathway is often associated with maintaining homeostasis in endocrine and exocrine cells.